D-glutamate(D-aspartate) oxidase activity [GO:0047819] (molecular function) Relationships: is a type of D-amino-acid oxidase activity [GO:0003884] Note: For the individual reactions, see instead 'D-glutamate oxidase activity ;GO:0047821' and 'D-aspartate oxidase activity ; GO:0008445'. Also known as: D-glutamate(D-aspartate):oxygen oxidoreductase (deaminating), D-glutamic-aspartic oxidase activity, D-monoaminodicarboxylic acid oxidase activity Definition: Catalysis of the reaction: D-glutamate + H2O + O2 = 2-oxoglutarate + NH3 + H2O2, and D-aspartate + H2O + O2 = oxaloacetate + NH3 + H2O2. Sources: EC:1.4.3.15